{
  "gene": "UniProtKB:Q96PD6",
  "term_label": "endoplasmic reticulum membrane",
  "term_id": "GO:0005789",
  "gene_symbol": "MOGAT1",
  "gene_name": "2-acylglycerol O-acyltransferase 1"
}